{
  "term_id": "GO:0000785",
  "term_label": "chromatin",
  "gene_symbol": "HNRNPAB",
  "gene": "UniProtKB:Q99729",
  "gene_name": "Heterogeneous nuclear ribonucleoprotein A_B"
}